antigen processing and presentation [GO:0019882] (biological process) Regulation: regulated by regulation of antigen processing and presentation [GO:0002577]; negatively regulated by GO:0002578; positively regulated by positive regulation of antigen processing and presentation [GO:0002579] Also known as: antigen presentation, antigen processing Relationships: is a type of immune system process [GO:0002376] Subtypes: B cell antigen processing and presentation [GO:0002450], T cell antigen processing and presentation [GO:0002457], GO:0002468, GO:0002471, macrophage antigen processing and presentation [GO:0002472], non-professional antigen presenting cell antigen processing and presentation [GO:0002473], antigen processing and presentation via MHC class Ib [GO:0002475], antigen processing and presentation of peptide or polysaccharide antigen via MHC class II [GO:0002504], antigen processing and presentation initiated by receptor mediated uptake of antigen [GO:0002745], antigen processing and presentation following pinocytosis [GO:0002746], GO:0002747, GO:0019883, antigen processing and presentation of exogenous antigen [GO:0019884], antigen processing and presentation of peptide antigen [GO:0048002] References: PMID:15771591, PMID:15928678 Sources: GOC:add, GO_REF:0000022, ISBN:0781735149 Definition: The process in which an antigen-presenting cell expresses antigen (peptide or lipid) on its cell surface in association with an MHC protein complex.